{
  "term_id": "GO:0045236",
  "gene_symbol": "PF4V1",
  "gene": "UniProtKB:P10720",
  "gene_name": "Platelet factor 4 variant",
  "term_label": "CXCR chemokine receptor binding"
}